branched-chain 2-oxo acid dehydrogenase activity [GO:0003863] (molecular function) Relationships: is a type of oxidoreductase activity, acting on the aldehyde or oxo group of donors, disulfide as acceptor [GO:0016624] Sources: EC:1.2.4.4 Also known as: 3-methyl-2-oxobutanoate dehydrogenase (2-methylpropanoyl-transferring) activity, alpha-ketoacid dehydrogenase activity, 2-oxoisocaproate dehydrogenase activity, 2-oxoisovalerate (lipoate) dehydrogenase activity, 3-methyl-2-oxobutanoate dehydrogenase (lipoamide) activity, 3-methyl-2-oxobutanoate:dihydrolipoyllysine-residue (2-methylpropanoyl)transferase-lipoyllysine 2-oxidoreductase (decarboxylating, acceptor-2-methylpropanoylating), 3-methyl-2-oxobutanoate:lipoamide oxidoreductase (decarboxylating and acceptor-2-methylpropanoylating) activity, BCKDH activity, BCOAD activity, alpha-keto-alpha-methylvalerate dehydrogenase activity, alpha-ketoisocaproate dehydrogenase activity, alpha-ketoisocaproic dehydrogenase activity, alpha-ketoisocaproic-alpha-keto-alpha-methylvaleric dehydrogenase activity, alpha-ketoisovalerate dehydrogenase activity, alpha-oxoisocaproate dehydrogenase activity, branched chain keto acid dehydrogenase activity, branched-chain (-2-oxoacid) dehydrogenase (BCD) activity, branched-chain 2-keto acid dehydrogenase activity, branched-chain alpha-keto acid dehydrogenase activity, branched-chain alpha-oxo acid dehydrogenase activity, branched-chain keto acid dehydrogenase activity, branched-chain ketoacid dehydrogenase activity, dehydrogenase, 2-oxoisovalerate (lipoate) activity, dehydrogenase, branched chain alpha-keto acid activity Definition: Catalysis of the reaction: N(6)-[(R)-lipoyl]-L-lysyl-[dihydrolipoyllysine-residue (2-methylpropanoyl)transferase] + 3-methyl-2-oxobutanoate + H+ = N(6)-[(R)-S(8)-2-methylpropanoyldihydrolipoyl]-L-lysyl-[dihydrolipoyllysine-residue (2-methylpropanoyl)transferase] + CO2. Also acts on 4-methyl-2-oxopentanoate and (S)-3-methyl-2-oxopentanoate, so that it acts on the 2-oxo acids that derive from the action of transaminases on valine, leucine and isoleucine.